{
  "gene_symbol": "NCLN",
  "term_id": "GO:0005789",
  "term_label": "endoplasmic reticulum membrane",
  "gene_name": "BOS complex subunit NCLN",
  "gene": "UniProtKB:Q969V3"
}